{
  "gene_name": "Thromboxane A2 receptor",
  "gene": "UniProtKB:P21731",
  "term_id": "GO:0045907",
  "gene_symbol": "TBXA2R",
  "term_label": "positive regulation of vasoconstriction"
}